{
  "term_label": "purine-nucleoside phosphorylase activity",
  "gene_symbol": "PNP",
  "term_id": "GO:0004731",
  "gene_name": "Purine nucleoside phosphorylase",
  "gene": "UniProtKB:P00491"
}